{
  "gene_symbol": "SETD9",
  "gene_name": "SET domain-containing protein 9",
  "term_label": "Unknown molecular function",
  "term_id": "UNKNOWN:0001",
  "gene": "UniProtKB:Q8NE22"
}